{
  "gene_name": "Microtubule-associated protein 10",
  "term_id": "GO:0030496",
  "gene": "UniProtKB:Q9P2G4",
  "gene_symbol": "MAP10",
  "term_label": "midbody"
}